{
  "gene_symbol": "GABRA4",
  "term_id": "GO:1904862",
  "gene_name": "Gamma-aminobutyric acid receptor subunit alpha-4",
  "gene": "UniProtKB:P48169",
  "term_label": "inhibitory synapse assembly"
}